mitochondrial mRNA processing [GO:0090615] (biological process) Subtypes: GO:0090616, mitochondrial mRNA 5'-end processing [GO:0090617] References: PMID:25181358 Sources: GOC:tb Definition: Steps involved in processing precursor RNAs arising from transcription of operons in the mitochondrial genome into mature mRNAs. Relationships: is a type of mitochondrial RNA metabolic process [GO:0000959]; is a type of mitochondrial RNA processing [GO:0000963]; is a type of mRNA processing [GO:0006397]